clathrin-coated pit [GO:0005905] (cellular component) Relationships: is a type of membrane [GO:0016020]; is part of GO:0012505 Also known as: coated pit References: PMID:10559856, PMID:17284835 Sources: GOC:mah, ISBN:0198506732, NIF_Subcellular:sao1969557946 Definition: A part of the endomembrane system in the form of an invagination of a membrane upon which a clathrin coat forms, and that can be converted by vesicle budding into a clathrin-coated vesicle. Coated pits form on the plasma membrane, where they are involved in receptor-mediated selective transport of many proteins and other macromolecules across the cell membrane, in the trans-Golgi network, and on some endosomes.